{
  "gene": "UniProtKB:Q92832",
  "gene_name": "Protein kinase C-binding protein NELL1",
  "term_label": "cytoplasm",
  "gene_symbol": "NELL1",
  "term_id": "GO:0005737"
}